{
  "term_id": "GO:0000978",
  "gene": "UniProtKB:P23759",
  "gene_name": "Paired box protein Pax-7",
  "gene_symbol": "PAX7",
  "term_label": "RNA polymerase II cis-regulatory region sequence-specific DNA binding"
}